{
  "gene_symbol": "SRRM4",
  "gene": "UniProtKB:A7MD48",
  "term_id": "GO:0042551",
  "term_label": "neuron maturation",
  "gene_name": "Serine_arginine repetitive matrix protein 4"
}